{
  "term_id": "GO:0008637",
  "gene": "UniProtKB:Q13323",
  "gene_name": "Bcl-2-interacting killer",
  "term_label": "apoptotic mitochondrial changes",
  "gene_symbol": "BIK"
}